regulation of RNA polymerase II regulatory region sequence-specific DNA binding [GO:1903025] (biological process) References: PMID:20026326 Sources: GOC:TermGenie, GOC:dph, GOC:krc, GO_REF:0000059 Subtypes: negative regulation of RNA polymerase II regulatory region sequence-specific DNA binding [GO:1903026] Definition: Any process that modulates the frequency, rate or extent of RNA polymerase II regulatory region sequence-specific DNA binding. Relationships: is a type of regulation of transcription regulatory region DNA binding [GO:2000677]; regulates RNA polymerase II transcription regulatory region sequence-specific DNA binding [GO:0000977]